{
  "term_id": "GO:0004383",
  "gene_symbol": "GUCY1B2",
  "term_label": "guanylate cyclase activity",
  "gene_name": "Guanylate cyclase soluble subunit beta-2",
  "gene": "UniProtKB:O75343"
}